{
  "term_label": "molybdenum ion binding",
  "gene_name": "Mitochondrial amidoxime-reducing component 1",
  "gene_symbol": "MTARC1",
  "gene": "UniProtKB:Q5VT66",
  "term_id": "GO:0030151"
}